pineal gland development [GO:0021982] (biological process) Relationships: is a type of GO:0048732; is part of diencephalon development [GO:0021536]; is part of endocrine system development [GO:0035270] Sources: GOC:cls, GOC:dgh, GOC:dph, GOC:jid, GO_REF:0000021 Also known as: epiphysis development Definition: The progression of the pineal gland over time from its initial formation until its mature state. The pineal gland is an endocrine gland that secretes melatonin and is involved in circadian rhythms.